{
  "gene": "UniProtKB:Q2KHN1",
  "term_id": "GO:0006511",
  "gene_symbol": "RNF151",
  "term_label": "ubiquitin-dependent protein catabolic process",
  "gene_name": "RING finger protein 151"
}